{
  "term_id": "GO:0005085",
  "gene": "UniProtKB:Q70Z35",
  "gene_name": "Phosphatidylinositol 3,4,5-trisphosphate-dependent Rac exchanger 2 protein",
  "gene_symbol": "PREX2",
  "term_label": "guanyl-nucleotide exchange factor activity"
}